{
  "term_id": "GO:0051560",
  "gene": "UniProtKB:Q9NWR8",
  "gene_name": "Calcium uniporter regulatory subunit MCUb, mitochondrial",
  "term_label": "mitochondrial calcium ion homeostasis",
  "gene_symbol": "MCUB"
}